{
  "gene": "UniProtKB:Q70EL3",
  "term_label": "cytosol",
  "gene_symbol": "USP50",
  "term_id": "GO:0005829",
  "gene_name": "Inactive ubiquitin carboxyl-terminal hydrolase 50"
}